{
  "term_id": "GO:0008284",
  "gene_symbol": "CSF2RA",
  "gene": "UniProtKB:P15509",
  "term_label": "positive regulation of cell population proliferation",
  "gene_name": "Granulocyte-macrophage colony-stimulating factor receptor subunit alpha"
}